cysteine-type carboxypeptidase activity [GO:0016807] (molecular function) Sources: GOC:mah, https://www.ebi.ac.uk/merops/about/glossary.shtml#CARBOXYPEPTIDASE Definition: Catalysis of the hydrolysis of a single C-terminal amino acid residue from a polypeptide chain by a mechanism in which the sulfhydryl group of a cysteine residue at the active center acts as a nucleophile. Relationships: is_a GO:0004180; is a type of cysteine-type exopeptidase activity [GO:0070004]